amino acid:proton symporter activity [GO:0005280] (molecular function) Definition: Enables the transfer of a solute or solutes from one side of a membrane to the other according to the reaction: amino acid(out) + H+(out) = amino acid(in) + H+(in). Subtypes: proline:proton symporter activity [GO:0005297], GO:0015492, lysine:proton symporter activity [GO:0015493], GO:0015495 Also known as: cation/amino acid symporter, hydrogen:amino acid symporter activity Relationships: is a type of amino acid:monoatomic cation symporter activity [GO:0005416]; is a type of solute:proton symporter activity [GO:0015295] Sources: GOC:ai